{
  "gene_symbol": "CSN2",
  "gene_name": "Beta-casein",
  "term_label": "extracellular space",
  "term_id": "GO:0005615",
  "gene": "UniProtKB:P05814"
}